{
  "gene_name": "Gamma-tubulin complex component 2",
  "term_id": "GO:0031122",
  "gene_symbol": "TUBGCP2",
  "term_label": "cytoplasmic microtubule organization",
  "gene": "UniProtKB:Q9BSJ2"
}